{
  "term_id": "UNKNOWN:0001",
  "gene_symbol": "KRTAP3-3",
  "term_label": "Unknown molecular function",
  "gene_name": "Keratin-associated protein 3-3",
  "gene": "UniProtKB:Q9BYR6"
}